{
  "term_label": "mRNA export from nucleus",
  "gene": "UniProtKB:Q13769",
  "gene_name": "THO complex subunit 5 homolog",
  "term_id": "GO:0006406",
  "gene_symbol": "THOC5"
}